{
  "gene_symbol": "TUBB2A",
  "term_label": "microtubule cytoskeleton organization",
  "term_id": "GO:0000226",
  "gene_name": "Tubulin beta-2A chain",
  "gene": "UniProtKB:Q13885"
}